alpha-1,4-glucan-protein synthase (ADP-forming) activity [GO:0047211] (molecular function) Also known as: 1,4alpha-glucan-protein synthase (ADP-forming) activity, ADP-glucose:protein 4-alpha-D-glucosyltransferase activity, ADPglucose:protein 4-alpha-D-glucosyltransferase activity, ADPglucose:protein glucosyltransferase activity, adenosine diphosphoglucose-protein glucosyltransferase activity Sources: EC:2.4.1.113, MetaCyc:2.4.1.113-RXN Definition: Catalysis of the reaction: ADP-D-glucose + protein = alpha-D-glucosyl-protein + ADP. Relationships: is a type of hexosyltransferase activity [GO:0016758]; is a type of catalytic activity, acting on a protein [GO:0140096]